{
  "term_label": "RNA polymerase II transcription regulatory region sequence-specific DNA binding",
  "gene_name": "ALX homeobox protein 1",
  "gene_symbol": "ALX1",
  "gene": "UniProtKB:Q15699",
  "term_id": "GO:0000977"
}